{
  "term_id": "GO:0007216",
  "gene": "UniProtKB:Q14833",
  "term_label": "G protein-coupled glutamate receptor signaling pathway",
  "gene_name": "Metabotropic glutamate receptor 4",
  "gene_symbol": "GRM4"
}